{
  "gene_name": "Membrane-spanning 4-domains subfamily A member 13",
  "term_id": "GO:0005886",
  "gene": "UniProtKB:Q5J8X5",
  "term_label": "plasma membrane",
  "gene_symbol": "MS4A13"
}